{
  "term_label": "Unknown cellular component",
  "gene": "UniProtKB:A6NI28",
  "gene_name": "Rho GTPase-activating protein 42",
  "term_id": "UNKNOWN:0003",
  "gene_symbol": "ARHGAP42"
}